purine nucleobase metabolic process [GO:0006144] (biological process) Definition: The chemical reactions and pathways involving purine nucleobases, one of the two classes of nitrogen-containing ring compounds found in DNA and RNA, which include adenine and guanine. Sources: GOC:go_curators Also known as: purine base metabolic process, purine base metabolism, purine metabolic process, purine metabolism Regulation: regulated by regulation of purine nucleobase metabolic process [GO:0006141]; negatively regulated by negative regulation of purine nucleobase metabolic process [GO:0045982]; positively regulated by positive regulation of purine nucleobase metabolic process [GO:0045983] Subtypes: purine nucleobase catabolic process [GO:0006145], purine nucleobase biosynthetic process [GO:0009113], adenine metabolic process [GO:0046083], GO:0046098, hypoxanthine metabolic process [GO:0046100], GO:0046110 Relationships: is_a nucleobase metabolic process [GO:0009112]; is a type of purine-containing compound metabolic process [GO:0072521]